arogenate dehydratase activity [GO:0047769] (molecular function) Definition: Catalysis of the reaction: L-arogenate = L-phenylalanine + H2O + CO2. Sources: EC:4.2.1.91 Also known as: carboxycyclohexadienyl dehydratase activity, L-arogenate hydro-lyase (decarboxylating), L-arogenate hydro-lyase (decarboxylating; L-phenylalanine-forming) Relationships: is a type of GO:0016836